{
  "term_id": "GO:0005737",
  "term_label": "cytoplasm",
  "gene_name": "G protein-coupled receptor kinase 4",
  "gene": "UniProtKB:P32298",
  "gene_symbol": "GRK4"
}